clathrin coat disassembly [GO:0072318] (biological process) References: PMID:11084334, PMID:11146663, PMID:8524399 Also known as: clathrin-coat disassembly, clathrin-coat uncoating, clathrin-coated vesicle uncoating Definition: The disaggregation of a clathrin coat into its constituent components; results in stripping or removing the clathrin coat from clathrin-coated vesicles (CCV) before fusing with their targets. CVVs transport cargo from plasma membrane and trans-Golgi to the endosomal system. Subtypes: synaptic vesicle uncoating [GO:0016191] Relationships: is_a vesicle uncoating [GO:0072319]